{
  "gene": "UniProtKB:Q00888",
  "gene_symbol": "PSG4",
  "gene_name": "Pregnancy-specific beta-1-glycoprotein 4",
  "term_id": "UNKNOWN:0002",
  "term_label": "Unknown biological process"
}